{
  "gene_symbol": "IPO8",
  "term_id": "GO:0005635",
  "term_label": "nuclear envelope",
  "gene_name": "Importin-8",
  "gene": "UniProtKB:O15397"
}